regulation of cholesterol storage [GO:0010885] (biological process) Definition: Any process that modulates the rate or extent of cholesterol storage. Cholesterol storage is the accumulation and maintenance in cells or tissues of cholesterol, cholest-5-en-3 beta-ol, the principal sterol of vertebrates and the precursor of many steroids, including bile acids and steroid hormones. Sources: GOC:BHF, GOC:dph, GOC:tb Relationships: is a type of regulation of lipid storage [GO:0010883]; regulates cholesterol storage [GO:0010878] Subtypes: GO:0010886, negative regulation of cholesterol storage [GO:0010887]